formaldehyde transketolase activity [GO:0047896] (molecular function) Relationships: is a type of transketolase or transaldolase activity [GO:0016744] Sources: EC:2.2.1.3, MetaCyc:FORMALDEHYDE-TRANSKETOLASE-RXN Definition: Catalysis of the reaction: D-xylulose 5-phosphate + formaldehyde = glyceraldehyde 3-phosphate + glycerone. Also known as: D-xylulose-5-phosphate:formaldehyde glycolaldehydetransferase activity, DHAS activity, dihydroxyacetone synthase activity, glycerone synthase activity